abscisic acid-activated signaling pathway involved in stomatal movement [GO:1901527] (biological process) Definition: Any abscisic acid mediated signaling pathway that is involved in stomatal movement. Relationships: is a type of GO:0009738; BFO_0000050 stomatal movement [GO:0010118] References: PMID:22730405 Sources: GOC:TermGenie Also known as: abscisic acid mediated signalling involved in stomatal movement, abscisic acid mediated signaling pathway involved in stomatal movement